racemase and epimerase activity, acting on amino acids and derivatives [GO:0016855] (molecular function) Sources: GOC:mah Subtypes: protein-serine epimerase activity [GO:0018365], isopenicillin-N epimerase activity [GO:0045439], 2-aminohexano-6-lactam racemase activity [GO:0047463], amino-acid racemase activity [GO:0047661], nocardicin-A epimerase activity [GO:0050143], L-Ala-D/L-Glu epimerase activity [GO:0103031] Relationships: is a type of GO:0016854 Definition: Catalysis of a reaction that alters the configuration of one or more chiral centers in an amino acid.